{
  "gene": "UniProtKB:Q8NEA6",
  "gene_name": "Zinc finger protein GLIS3",
  "term_id": "GO:0000981",
  "term_label": "DNA-binding transcription factor activity, RNA polymerase II-specific",
  "gene_symbol": "GLIS3"
}